{
  "gene_name": "Transcription cofactor vestigial-like protein 3",
  "term_id": "GO:0005634",
  "gene": "UniProtKB:A8MV65",
  "term_label": "nucleus",
  "gene_symbol": "VGLL3"
}